melanosome organization [GO:0032438] (biological process) Definition: A process that is carried out at the cellular level which results in the assembly, arrangement of constituent parts, or disassembly of a melanosome. A melanosome is a tissue-specific, membrane-bounded cytoplasmic organelle within which melanin pigments are synthesized and stored. Sources: GOC:vk Subtypes: melanosome assembly [GO:1903232] Regulation: regulated by GO:1903056; negatively regulated by negative regulation of melanosome organization [GO:1903057]; positively regulated by positive regulation of melanosome organization [GO:1903058] Also known as: melanosome organisation, melanosome organization and biogenesis Relationships: is a type of pigment granule organization [GO:0048753]